{
  "term_label": "regulation of cell migration",
  "term_id": "GO:0030334",
  "gene": "UniProtKB:Q9GZV9",
  "gene_name": "Fibroblast growth factor 23",
  "gene_symbol": "FGF23"
}